cotyledon morphogenesis [GO:0048826] (biological process) Definition: The process in which the anatomical structures of the cotyledon are generated and organized. The cotyledon is the modified leaf (seed leaf), found as part of the embryo in plant seeds. It is involved in either storage or absorption of food reserves. Dicotyledonous seeds contain two cotyledons, while monocotyledonous seeds contain only one. The cotyledons may appear above ground and show photosynthetic activity in the seedling. Relationships: is_a leaf morphogenesis [GO:0009965]; is a type of GO:0048598; is a type of post-embryonic plant morphogenesis [GO:0090698]; is part of cotyledon development [GO:0048825] Sources: GOC:devbiol, GOC:tb, PO:0020030